{
  "term_label": "Unknown cellular component",
  "gene_symbol": "C5orf24",
  "gene_name": "UPF0461 protein C5orf24",
  "gene": "UniProtKB:Q7Z6I8",
  "term_id": "UNKNOWN:0003"
}